{
  "term_id": "UNKNOWN:0003",
  "gene_name": "RWD domain-containing protein 4",
  "gene_symbol": "RWDD4",
  "term_label": "Unknown cellular component",
  "gene": "UniProtKB:Q6NW29"
}